{
  "term_id": "UNKNOWN:0003",
  "term_label": "Unknown cellular component",
  "gene_name": "Transmembrane and coiled-coil domain-containing protein 5A",
  "gene_symbol": "TMCO5A",
  "gene": "UniProtKB:Q8N6Q1"
}